{
  "term_label": "establishment or maintenance of epithelial cell apical/basal polarity",
  "gene_symbol": "CRB1",
  "gene": "UniProtKB:P82279",
  "term_id": "GO:0045197",
  "gene_name": "Protein crumbs homolog 1"
}